{
  "gene": "UniProtKB:Q96QA5",
  "term_label": "phosphatidylinositol-4,5-bisphosphate binding",
  "term_id": "GO:0005546",
  "gene_name": "Gasdermin-A",
  "gene_symbol": "GSDMA"
}